{
  "gene_name": "RNA exonuclease 4",
  "gene": "UniProtKB:Q9GZR2",
  "gene_symbol": "REXO4",
  "term_id": "GO:0006308",
  "term_label": "DNA catabolic process"
}